{
  "gene_name": "Retinoblastoma-like protein 1",
  "term_label": "cell differentiation",
  "gene_symbol": "RBL1",
  "gene": "UniProtKB:P28749",
  "term_id": "GO:0030154"
}